{
  "term_id": "UNKNOWN:0002",
  "gene": "UniProtKB:O43895",
  "gene_name": "Xaa-Pro aminopeptidase 2",
  "gene_symbol": "XPNPEP2",
  "term_label": "Unknown biological process"
}